{
  "gene_name": "Homeobox protein DLX-3",
  "gene_symbol": "DLX3",
  "term_label": "DNA-binding transcription factor activity, RNA polymerase II-specific",
  "term_id": "GO:0000981",
  "gene": "UniProtKB:O60479"
}